{
  "gene_name": "Homeobox protein Hox-A4",
  "gene": "UniProtKB:Q00056",
  "gene_symbol": "HOXA4",
  "term_label": "positive regulation of transcription by RNA polymerase II",
  "term_id": "GO:0045944"
}